{
  "gene": "UniProtKB:P56282",
  "gene_symbol": "POLE2",
  "gene_name": "DNA polymerase epsilon subunit 2",
  "term_id": "GO:0042276",
  "term_label": "error-prone translesion synthesis"
}